{
  "gene_name": "Myosin-4",
  "term_label": "actin filament binding",
  "gene": "UniProtKB:Q9Y623",
  "term_id": "GO:0051015",
  "gene_symbol": "MYH4"
}